endoplasmic reticulum exit site [GO:0070971] (cellular component) References: PMID:15623529, PMID:16957052 Sources: NIF_Subcellular:sao124393998 Definition: An endoplasmic reticulum part at which COPII-coated vesicles are produced. Also known as: ER exit site, transitional ER Relationships: is a type of cellular anatomical structure [GO:0110165]; is part of GO:0005783